phosphogluconate 2-dehydrogenase activity [GO:0008114] (molecular function) Also known as: 6-phosphogluconic dehydrogenase activity, 6-phosphogluconate 2-dehydrogenase activity, 2-keto-6-phosphogluconate reductase activity, 6-phospho-D-gluconate:NAD(P)+ 2-oxidoreductase activity, 6-phosphogluconate dehydrogenase (NAD), gluconate 6-phosphate dehydrogenase activity, phosphogluconate dehydrogenase activity Definition: Catalysis of the reaction: 6-phospho-D-gluconate + NADP+ = 6-phospho-2-dehydro-D-gluconate + NADPH. Sources: EC:1.1.1.43 Relationships: is a type of oxidoreductase activity, acting on the CH-OH group of donors, NAD or NADP as acceptor [GO:0016616]